{
  "term_id": "UNKNOWN:0003",
  "gene_name": "Sperm-tail PG-rich repeat-containing protein 2",
  "gene_symbol": "STPG2",
  "gene": "UniProtKB:Q8N412",
  "term_label": "Unknown cellular component"
}